negative regulation of fibroblast growth factor receptor signaling pathway involved in neural plate anterior/posterior pattern formation [GO:2000314] (biological process) Also known as: negative regulation of fibroblast growth factor receptor signalling pathway involved in neural plate anterior/posterior pattern formation Sources: GOC:BHF Relationships: is a type of negative regulation of fibroblast growth factor receptor signaling pathway [GO:0040037]; is a type of negative regulation of developmental process [GO:0051093]; is a type of GO:2000313; negatively regulates fibroblast growth factor receptor signaling pathway involved in neural plate anterior/posterior pattern formation [GO:0060825] Definition: Any process that stops, prevents or reduces the frequency, rate or extent of fibroblast growth factor receptor signaling pathway involved in neural plate anterior/posterior pattern formation.